{
  "gene_name": "Tubulin polymerization-promoting protein family member 2",
  "gene_symbol": "TPPP2",
  "term_id": "GO:0015631",
  "gene": "UniProtKB:P59282",
  "term_label": "tubulin binding"
}